acid phosphatase complex [GO:1904097] (CC) Relationships: is a type of phosphatase complex [GO:1903293] Definition: A protein complex which is capable of acid phosphatase activity. Note: An example of this is ACPP in human (UniProt symbol P15309) in PMID:22389722 (inferred from physical interaction). References: PMID:8132635 Sources: GOC:TermGenie, GOC:bhm, GO_REF:0000088